somatic cell DNA recombination [GO:0016444] (biological process) Relationships: is a type of DNA recombination [GO:0006310] Subtypes: somatic diversification of immune receptors via germline recombination within a single locus [GO:0002562], somatic diversification of immune receptors via gene conversion [GO:0002565] Sources: GOC:ma Definition: Recombination occurring within or between DNA molecules in somatic cells.